{
  "gene_symbol": "ATP1A1-AS1",
  "gene_name": "Putative uncharacterized protein ATP1A1-AS1",
  "term_id": "UNKNOWN:0002",
  "gene": "UniProtKB:Q5TC04",
  "term_label": "Unknown biological process"
}